regulation of synaptic transmission, GABAergic [GO:0032228] (biological process) Definition: Any process that modulates the frequency, rate or extent of GABAergic synaptic transmission, the process of communication from a neuron to another neuron across a synapse using the neurotransmitter gamma-aminobutyric acid (GABA). Relationships: is a type of modulation of chemical synaptic transmission [GO:0050804]; regulates GO:0051932 Sources: GOC:mah Subtypes: negative regulation of synaptic transmission, GABAergic [GO:0032229], positive regulation of synaptic transmission, GABAergic [GO:0032230]